{
  "term_label": "Unknown biological process",
  "gene_name": "Protein kinase C-binding protein NELL2",
  "gene_symbol": "NELL2",
  "term_id": "UNKNOWN:0002",
  "gene": "UniProtKB:Q99435"
}